{
  "gene_symbol": "LINC00479",
  "term_id": "UNKNOWN:0003",
  "gene_name": "Putative uncharacterized protein encoded by LINC00479",
  "gene": "UniProtKB:Q96M42",
  "term_label": "Unknown cellular component"
}